fermentative hydrogen production [GO:0044812] (BP) Definition: The fermentation of organic substances with a net release of hydrogen. Also known as: carbohydrate fermentation Sources: GOC:mengo_curators Relationships: is a type of GO:0006113; is a type of GO:1902422